{
  "gene_symbol": "ITGB8",
  "term_label": "integrin complex",
  "gene_name": "Integrin beta-8",
  "term_id": "GO:0008305",
  "gene": "UniProtKB:P26012"
}